{
  "term_label": "Unknown molecular function",
  "gene_name": "Immunoglobulin superfamily member 5",
  "gene": "UniProtKB:Q9NSI5",
  "term_id": "UNKNOWN:0001",
  "gene_symbol": "IGSF5"
}